L-histidine catabolic process to glutamate and formate [GO:0019557] (biological process) Sources: GOC:go_curators Definition: The chemical reactions and pathways resulting in the breakdown of L-histidine into other compounds, including glutamate and formate. Also known as: histidine catabolic process to glutamate and formate, histidine breakdown to glutamate and formate, histidine degradation to glutamate and formate Relationships: is a type of glutamate metabolic process [GO:0006536]; is a type of GO:0006548; is a type of formate metabolic process [GO:0015942]